{
  "term_label": "cell morphogenesis",
  "gene_symbol": "CDH15",
  "gene": "UniProtKB:P55291",
  "gene_name": "Cadherin-15",
  "term_id": "GO:0000902"
}